{
  "gene_name": "H_ACA ribonucleoprotein complex non-core subunit NAF1",
  "term_label": "sno(s)RNA-containing ribonucleoprotein complex",
  "gene_symbol": "NAF1",
  "term_id": "GO:0005732",
  "gene": "UniProtKB:Q96HR8"
}